{
  "gene_symbol": "SHARPIN",
  "gene_name": "Sharpin",
  "term_label": "positive regulation of canonical NF-kappaB signal transduction",
  "gene": "UniProtKB:Q9H0F6",
  "term_id": "GO:0043123"
}